{
  "gene_name": "Potassium-transporting ATPase subunit beta",
  "term_label": "sodium:potassium-exchanging ATPase complex",
  "gene_symbol": "ATP4B",
  "gene": "UniProtKB:P51164",
  "term_id": "GO:0005890"
}